{
  "gene_name": "Fibroblast growth factor receptor-like 1",
  "term_id": "GO:0005007",
  "gene_symbol": "FGFRL1",
  "gene": "UniProtKB:Q8N441",
  "term_label": "fibroblast growth factor receptor activity"
}